{
  "term_id": "UNKNOWN:0001",
  "gene_symbol": "A0A6Q8PFC9",
  "gene_name": "Uncharacterized protein",
  "term_label": "Unknown molecular function",
  "gene": "UniProtKB:A0A6Q8PFC9"
}